{
  "gene_symbol": "SAMD8",
  "term_label": "Golgi membrane",
  "gene": "UniProtKB:Q96LT4",
  "gene_name": "Sphingomyelin synthase-related protein 1",
  "term_id": "GO:0000139"
}